{
  "term_label": "G protein-coupled purinergic nucleotide receptor activity",
  "gene_symbol": "GPR171",
  "gene": "UniProtKB:O14626",
  "gene_name": "G-protein coupled receptor 171",
  "term_id": "GO:0045028"
}